{
  "term_label": "poly(A)-dependent snoRNA 3'-end processing",
  "term_id": "GO:0071051",
  "gene": "UniProtKB:Q9NQT4",
  "gene_symbol": "EXOSC5",
  "gene_name": "Exosome complex component RRP46"
}